{
  "gene_name": "Actin-related protein 8",
  "gene": "UniProtKB:Q9H981",
  "term_id": "GO:0006302",
  "gene_symbol": "ACTR8",
  "term_label": "double-strand break repair"
}